{
  "gene_symbol": "ZRSR2",
  "gene": "UniProtKB:Q15696",
  "gene_name": "U2 small nuclear ribonucleoprotein auxiliary factor 35 kDa subunit-related protein 2",
  "term_id": "GO:0000398",
  "term_label": "mRNA splicing, via spliceosome"
}